mesonephric glomerular epithelial cell development [GO:0061251] (BP) Relationships: is a type of glomerular epithelial cell development [GO:0072310]; is part of GO:0061250 Sources: GOC:mtg_kidney_jan10 Definition: The process whose specific outcome is the progression of a mesonephric glomerular epithelial cell over time, from its formation to the mature structure. Mesonephric glomerular epithelial cells are specialized epithelial cells that form part of the mesonephric glomerulus; there are two types, mesonephric glomerular parietal epithelial cells and mesonephric glomerular visceral epithelial cells. Subtypes: mesonephric glomerular parietal epithelial cell development [GO:0061254], mesonephric podocyte development [GO:0061257], GO:0061258